{
  "gene_name": "Ena_VASP-like protein",
  "term_id": "GO:0030838",
  "gene": "UniProtKB:Q9UI08",
  "gene_symbol": "EVL",
  "term_label": "positive regulation of actin filament polymerization"
}